{
  "gene_name": "tRNA modification GTPase GTPBP3, mitochondrial",
  "term_id": "GO:0030488",
  "gene_symbol": "GTPBP3",
  "term_label": "tRNA methylation",
  "gene": "UniProtKB:Q969Y2"
}